{
  "term_id": "GO:0048487",
  "gene": "UniProtKB:Q6TDU7",
  "gene_symbol": "DNAI7",
  "gene_name": "Dynein axonemal intermediate chain 7",
  "term_label": "beta-tubulin binding"
}